negative regulation of SREBP signaling pathway [GO:2000639] (biological process) Subtypes: GO:0036316, negative regulation of SREBP signaling pathway in response to increased oxygen levels [GO:0038175] Relationships: is a type of GO:1902532; is a type of GO:2000638; negatively regulates SREBP signaling pathway [GO:0032933] Sources: GOC:BHF Definition: Any process that stops, prevents or reduces the frequency, rate or extent of the SREBP signaling pathway. Also known as: negative regulation of SREBP-mediated signaling pathway, negative regulation of SREBP-mediated signalling pathway